{
  "gene_symbol": "LTA",
  "term_id": "GO:0005615",
  "gene": "UniProtKB:P01374",
  "term_label": "extracellular space",
  "gene_name": "Lymphotoxin-alpha"
}